glial cell fate commitment [GO:0021781] (biological process) Definition: The process in which the developmental fate of a cell becomes restricted such that it will develop into a glial cell. Sources: GOC:cls, GOC:dgh, GOC:dph, GOC:jid, GO_REF:0000021 Relationships: is a type of GO:0045165; is part of glial cell differentiation [GO:0010001] Subtypes: oligodendrocyte cell fate commitment [GO:0021779], radial glial cell fate commitment in forebrain [GO:0022023], GO:0060018, cardiac glial cell fate commitment [GO:0060953]